arachidonate 8(S)-lipoxygenase activity [GO:0036403] (molecular function) Relationships: is a type of oxidoreductase activity, acting on single donors with incorporation of molecular oxygen, incorporation of two atoms of oxygen [GO:0016702] References: PMID:10625675 Sources: GOC:lb, RHEA:38675 Definition: Catalysis of the reaction: arachidonate + O2 = (5Z,8S,9E,11Z,14Z)-8-hydroperoxyicosa-5,9,11,14-tetraenoate. Note: This activity produces the S-enantiomer of HPETE, 8(S)-HPETE. For the reaction producing the S-enantiomer, see GO:0047677. Also known as: 8(S)-lipoxygenase activity, 8-lipoxygenase (S-type)